tRNA-guanine transglycosylase complex [GO:0120507] (cellular component) Also known as: TGT, queuine tRNA-ribosyltransferase complex References: PMID:20354154, PMID:38181786 Sources: GOC:sjm Relationships: is a type of GO:1990234 Definition: A protein complex that catalyzes the base-exchange of a guanine residue with queuine at the wobble position of the anticodon of tRNAs. The eukaryotic tRNA-guanine transglycosylase exists as a heterodimer of a catalytic subunit (QTRT1 in humans) and an accessory subunit (QTRT2 in humans), whereas the bacterial enzyme is homodimeric.